{
  "term_id": "UNKNOWN:0001",
  "gene_name": "Proline-rich protein 32",
  "gene_symbol": "PRR32",
  "term_label": "Unknown molecular function",
  "gene": "UniProtKB:B1ATL7"
}